{
  "gene_name": "Bcl-2-like protein 15",
  "term_label": "cytosol",
  "gene_symbol": "BCL2L15",
  "gene": "UniProtKB:Q5TBC7",
  "term_id": "GO:0005829"
}